alpha-amylase activity [GO:0004556] (molecular function) Definition: Catalysis of the endohydrolysis of (1->4)-alpha-D-glucosidic linkages in polysaccharides containing three or more alpha-(1->4)-linked D-glucose units. References: PMID:12527308 Also known as: glycogenase activity, alpha-amylase activity (releasing maltohexaose), 1,4-alpha-D-glucan glucanohydrolase activity, alpha amylase activity, endoamylase activity, taka-amylase A Relationships: is_a amylase activity [GO:0016160] Regulation: negatively regulated by alpha-amylase inhibitor activity [GO:0015066]